UDP-glucose:hexose-1-phosphate uridylyltransferase activity [GO:0008108] (molecular function) Sources: EC:2.7.7.12, RHEA:13989 Definition: Catalysis of the reaction: alpha-D-galactose 1-phosphate + UDP-D-glucose = alpha-D-glucose 1-phosphate + UDP-D-galactose. Also known as: Gal-1-P uridylyltransferase activity, galactose-1-phosphate uridylyltransferase activity, uridyl transferase activity, uridyltransferase activity, uridylyl removing enzyme activity, UDP-glucose-hexose-1-phosphate uridylyltransferase activity, UDP-glucose:alpha-D-galactose-1-phosphate uridylyltransferase activity, UDPglucose-hexose-1-phosphate uridylyltransferase activity, UDPglucose:alpha-D-galactose-1-phosphate uridylyltransferase activity, hexose 1-phosphate uridyltransferase activity, hexose-1-phosphate uridylyltransferase activity Relationships: is a type of uridylyltransferase activity [GO:0070569]